{
  "term_id": "GO:0032006",
  "term_label": "regulation of TOR signaling",
  "gene_symbol": "ROS1",
  "gene_name": "Proto-oncogene tyrosine-protein kinase ROS",
  "gene": "UniProtKB:P08922"
}